{
  "term_id": "GO:0005509",
  "gene": "UniProtKB:Q14573",
  "gene_symbol": "ITPR3",
  "term_label": "calcium ion binding",
  "gene_name": "Inositol 1,4,5-trisphosphate receptor type 3"
}